{
  "term_label": "Unknown biological process",
  "gene_symbol": "DNAJC14",
  "gene": "UniProtKB:Q6Y2X3",
  "term_id": "UNKNOWN:0002",
  "gene_name": "DnaJ homolog subfamily C member 14"
}